TTP metabolic process [GO:0046046] (biological process) Subtypes: TTP biosynthetic process [GO:0006234], GO:0046047 Also known as: TTP metabolism Relationships: is a type of pyrimidine ribonucleoside triphosphate metabolic process [GO:0009208]; is a type of pyrimidine ribonucleotide metabolic process [GO:0009218] Sources: GOC:go_curators Definition: The chemical reactions and pathways involving TTP, ribosylthymine triphosphate.